cell movement involved in somal translocation [GO:0021805] (biological process) Definition: The movement of a cell body from the ventricular zone to the pial surface with a concomitant shortening of the process that extends to the pial surface. References: PMID:12626695 Sources: GOC:cls, GOC:dgh, GOC:dph, GOC:jid, GO_REF:0000021 Also known as: cell motility involved in somal translocation Relationships: is a type of cell motility [GO:0048870]; is part of somal translocation [GO:0021802]